{
  "term_id": "GO:0047522",
  "gene_symbol": "PTGR1",
  "gene": "UniProtKB:Q14914",
  "gene_name": "Prostaglandin reductase 1",
  "term_label": "15-oxoprostaglandin 13-reductase [NAD(P)+] activity"
}